{
  "gene_name": "Pleckstrin homology domain-containing family J member 1",
  "gene_symbol": "PLEKHJ1",
  "gene": "UniProtKB:Q9NW61",
  "term_label": "early endosome",
  "term_id": "GO:0005769"
}